{
  "gene": "UniProtKB:Q15072",
  "gene_name": "Zinc finger protein OZF",
  "term_label": "regulation of transcription by RNA polymerase II",
  "term_id": "GO:0006357",
  "gene_symbol": "ZNF146"
}